clathrin-dependent endocytosis involved in vitellogenesis [GO:0061883] (biological process) Also known as: clathrin-dependent endocytosis involved in yolk formation Relationships: is a type of clathrin-dependent endocytosis [GO:0072583]; is part of vitellogenesis [GO:0007296] References: PMID:26265702 Definition: A clathrin-mediated endocytosis process whereby yolk proteins are internalized and trafficked through the endocytic pathway for yolk deposition.